{
  "gene": "UniProtKB:P01569",
  "term_id": "GO:0006959",
  "gene_name": "Interferon alpha-5",
  "gene_symbol": "IFNA5",
  "term_label": "humoral immune response"
}